{
  "term_id": "UNKNOWN:0003",
  "term_label": "Unknown cellular component",
  "gene_name": "Late cornified envelope protein 2B",
  "gene_symbol": "LCE2B",
  "gene": "UniProtKB:O14633"
}